{
  "term_id": "GO:0006357",
  "gene_symbol": "ZNF728",
  "term_label": "regulation of transcription by RNA polymerase II",
  "gene": "UniProtKB:P0DKX0",
  "gene_name": "Zinc finger protein 728"
}